{
  "gene_symbol": "CABP2",
  "term_id": "GO:0007601",
  "gene": "UniProtKB:Q9NPB3",
  "term_label": "visual perception",
  "gene_name": "Calcium-binding protein 2"
}